response to temperature stimulus [GO:0009266] (biological process) Relationships: is a type of response to abiotic stimulus [GO:0009628] Also known as: response to thermal stimulus Subtypes: response to heat [GO:0009408], response to cold [GO:0009409], temperature compensation of the circadian clock [GO:0010378], detection of temperature stimulus [GO:0016048], thermosensory behavior [GO:0040040], thermotaxis [GO:0043052], cellular response to temperature stimulus [GO:0071502], GO:0140919 Sources: GOC:hb Definition: Any process that results in a change in state or activity of a cell or an organism (in terms of movement, secretion, enzyme production, gene expression, etc.) as a result of a temperature stimulus.